{
  "gene": "UniProtKB:P50851",
  "gene_name": "Lipopolysaccharide-responsive and beige-like anchor protein",
  "term_label": "membrane",
  "gene_symbol": "LRBA",
  "term_id": "GO:0016020"
}